{
  "term_id": "UNKNOWN:0001",
  "gene": "UniProtKB:A0A1B0GUT2",
  "gene_name": "Uncharacterized protein C10orf143",
  "gene_symbol": "C10orf143",
  "term_label": "Unknown molecular function"
}